ribosome binding [GO:0043022] (molecular function) Relationships: is a type of ribonucleoprotein complex binding [GO:0043021] Also known as: ribosome receptor activity Sources: GOC:go_curators Subtypes: ribosomal large subunit binding [GO:0043023], ribosomal small subunit binding [GO:0043024], mitochondrial ribosome binding [GO:0097177] Definition: Binding to a ribosome.